bulbus arteriosus morphogenesis [GO:0003233] (biological process) Relationships: is a type of cardiac chamber morphogenesis [GO:0003206]; is part of GO:0003232 Sources: GOC:mtg_heart Definition: The process in which the bulbus arteriosus is generated and organized. The bulbus arteriosus is an elastic cardiac chamber.